hypoglossal nucleus development [GO:0021743] (biological process) Definition: The process whose specific outcome is the progression of the hypoglossal nucleus over time, from its formation to the mature structure. Relationships: is a type of neural nucleus development [GO:0048857]; is part of medulla oblongata development [GO:0021550] Sources: GOC:cls, GOC:curators, GOC:dgh, GOC:dph, GOC:jid